positive regulation of cartilage condensation [GO:1902027] (biological process) Relationships: is_a positive regulation of cellular process [GO:0048522]; is a type of regulation of cartilage condensation [GO:1902026]; positively regulates cartilage condensation [GO:0001502] References: PMID:17202865 Sources: GOC:TermGenie Definition: Any process that activates or increases the frequency, rate or extent of cartilage condensation. Also known as: up regulation of cartilage condensation, up-regulation of cartilage condensation, upregulation of cartilage condensation, activation of cartilage condensation